{
  "gene_symbol": "FARSA",
  "term_label": "phenylalanine-tRNA ligase activity",
  "term_id": "GO:0004826",
  "gene": "UniProtKB:Q9Y285",
  "gene_name": "Phenylalanine--tRNA ligase alpha subunit"
}